cytoplasmic translational initiation [GO:0002183] (BP) Relationships: is a type of GO:0006413; is part of cytoplasmic translation [GO:0002181] Regulation: regulated by regulation of cytoplasmic translational initiation [GO:1904688]; negatively regulated by negative regulation of cytoplasmic translational initiation [GO:1904689]; positively regulated by positive regulation of cytoplasmic translational initiation [GO:1904690] Definition: The process preceding formation of the peptide bond between the first two amino acids of a protein in the cytoplasm. This includes the formation of a complex of the ribosome, mRNA or circRNA, and an initiation complex that contains the first aminoacyl-tRNA. Subtypes: translation reinitiation [GO:0002188], cap-independent translational initiation [GO:0002190], cap-dependent translational initiation [GO:0002191] Sources: GOC:hjd